{
  "term_id": "GO:0048706",
  "gene_name": "Homeobox protein DLX-1",
  "gene_symbol": "DLX1",
  "gene": "UniProtKB:P56177",
  "term_label": "embryonic skeletal system development"
}